negative regulation of bud outgrowth involved in lung branching [GO:0061112] (BP) Definition: Any process that decreases the rate, frequency, or extent of bud outgrowth involved in lung branching. Sources: GOC:dph Relationships: is a type of GO:0048640; is a type of negative regulation of branching involved in lung morphogenesis [GO:0061048]; negatively regulates bud outgrowth involved in lung branching [GO:0060447]